lamellipodium membrane [GO:0031258] (cellular component) Relationships: is a type of cell projection membrane [GO:0031253]; is a type of GO:0031256; is part of lamellipodium [GO:0030027] Sources: GOC:mah Definition: The portion of the plasma membrane surrounding a lamellipodium.